glucomannan 4-beta-mannosyltransferase activity [GO:0047259] (molecular function) Sources: EC:2.4.1.32, MetaCyc:2.4.1.32-RXN Also known as: GDP-mannose:glucomannan 1,4-beta-D-mannosyltransferase activity, glucomannan 4-b-mannosyltransferase activity, glucomannan-synthase activity, GDP-man-beta-mannan mannosyltransferase activity Relationships: is a type of beta-1,4-mannosyltransferase activity [GO:0019187] Definition: Catalysis of the reaction: glucomannan(n) + GDP-mannose = glucomannan(n+1) + GDP.